double-stranded DNA exodeoxyribonuclease activity [GO:0008309] (MF) Relationships: is_a GO:0016895 Subtypes: GO:0008311, double-stranded DNA 5'-3' DNA exonuclease activity [GO:0051908] Also known as: double-stranded DNA specific exodeoxyribonuclease activity Sources: GOC:mah Definition: Catalysis of the sequential cleavage of mononucleotides from a free 5' or 3' terminus of a double-stranded DNA molecule.